{
  "gene": "UniProtKB:P19484",
  "term_id": "GO:0006357",
  "gene_symbol": "TFEB",
  "term_label": "regulation of transcription by RNA polymerase II",
  "gene_name": "Transcription factor EB"
}